{
  "gene_name": "Zinc fingers and homeoboxes protein 3",
  "term_id": "GO:0005634",
  "gene": "UniProtKB:Q9H4I2",
  "gene_symbol": "ZHX3",
  "term_label": "nucleus"
}